{
  "gene_symbol": "OR52L2P",
  "gene_name": "Putative olfactory receptor 52L2",
  "gene": "UniProtKB:Q8NGH6",
  "term_label": "plasma membrane",
  "term_id": "GO:0005886"
}